positive regulation of kainate selective glutamate receptor signaling pathway [GO:0106428] (biological process) References: PMID:12597860 Relationships: is a type of positive regulation of biological process [GO:0048518]; is_a regulation of kainate selective glutamate receptor signaling pathway [GO:0106426]; positively regulates regulation of kainate selective glutamate receptor signaling pathway [GO:0106426] Definition: Any process that activates or increases the frequency, rate or extent of the kainate selective glutamate receptor signaling pathway.